{
  "gene_name": "Prothrombin",
  "gene_symbol": "F2",
  "gene": "UniProtKB:P00734",
  "term_id": "GO:0030194",
  "term_label": "positive regulation of blood coagulation"
}